{
  "term_label": "Unknown molecular function",
  "term_id": "UNKNOWN:0001",
  "gene_symbol": "C11orf52",
  "gene": "UniProtKB:Q96A22",
  "gene_name": "Uncharacterized protein C11orf52"
}